{
  "gene_symbol": "LCE1E",
  "gene": "UniProtKB:Q5T753",
  "term_id": "UNKNOWN:0002",
  "gene_name": "Late cornified envelope protein 1E",
  "term_label": "Unknown biological process"
}